glycolate dehydrogenase activity [GO:0019154] (molecular function) Relationships: is a type of oxidoreductase activity, acting on CH-OH group of donors [GO:0016614] Sources: EC:1.1.99.14, RHEA:21264 Also known as: glycolate oxidoreductase activity, glycolate:(acceptor) 2-oxidoreductase activity, glycolate:acceptor 2-oxidoreductase activity, glycolic acid dehydrogenase activity Definition: Catalysis of the reaction: A + glycolate = AH(2) + glyoxylate.